negative regulation of wound healing [GO:0061045] (biological process) Relationships: is a type of negative regulation of response to external stimulus [GO:0032102]; is a type of regulation of wound healing [GO:0061041]; is a type of negative regulation of response to wounding [GO:1903035]; negatively regulates wound healing [GO:0042060] Sources: GOC:dph Definition: Any process that decreases the rate, frequency, or extent of the series of events that restore integrity to a damaged tissue, following an injury. Subtypes: negative regulation of blood coagulation [GO:0030195], negative regulation of skeletal muscle tissue regeneration [GO:0043417], negative regulation of vascular wound healing [GO:0061044], negative regulation of wound healing, spreading of epidermal cells [GO:1903690], GO:1905685